{
  "term_label": "spliceosomal complex",
  "term_id": "GO:0005681",
  "gene_symbol": "U2AF1L4",
  "gene": "UniProtKB:Q8WU68",
  "gene_name": "Splicing factor U2AF 26 kDa subunit"
}